{
  "term_id": "GO:0008139",
  "gene_symbol": "KPNA3",
  "gene": "UniProtKB:O00505",
  "gene_name": "Importin subunit alpha-4",
  "term_label": "nuclear localization sequence binding"
}